{
  "term_label": "Unknown biological process",
  "gene_name": "Protein FAM24A",
  "gene": "UniProtKB:A6NFZ4",
  "term_id": "UNKNOWN:0002",
  "gene_symbol": "FAM24A"
}